regulation of systemic arterial blood pressure by ischemic conditions [GO:0001980] (biological process) Also known as: ischemic regulation of systemic arterial blood pressure, CNS ischemic response, ischemic control of blood pressure Definition: The process that modulates blood pressure by the detection of carbon dioxide levels in the brain stem. Increased levels activate the sympathetic vasoconstrictor mechanism increasing the force with which blood flows through the circulatory system. Sources: GOC:dph, GOC:tb, ISBN:0721643949 Relationships: is a type of nervous system process involved in regulation of systemic arterial blood pressure [GO:0001976]